{
  "term_id": "GO:0005085",
  "gene": "UniProtKB:Q92556",
  "term_label": "guanyl-nucleotide exchange factor activity",
  "gene_name": "Engulfment and cell motility protein 1",
  "gene_symbol": "ELMO1"
}